{
  "gene_symbol": "HMGXB3",
  "gene_name": "HMG domain-containing protein 3",
  "gene": "UniProtKB:Q12766",
  "term_id": "UNKNOWN:0002",
  "term_label": "Unknown biological process"
}